{
  "term_id": "GO:0005869",
  "gene": "UniProtKB:P42025",
  "gene_name": "Beta-centractin",
  "gene_symbol": "ACTR1B",
  "term_label": "dynactin complex"
}